{
  "term_id": "GO:0005886",
  "gene_name": "SHC-transforming protein 1",
  "term_label": "plasma membrane",
  "gene": "UniProtKB:P29353",
  "gene_symbol": "SHC1"
}